{
  "gene": "UniProtKB:Q8TEZ7",
  "gene_symbol": "PAQR8",
  "term_id": "GO:0005496",
  "gene_name": "Membrane progestin receptor beta",
  "term_label": "steroid binding"
}